ovarian follicle atresia [GO:0001552] (biological process) References: PMID:18638134 Sources: GOC:mtg_apoptosis Definition: A periodic process in which immature ovarian follicles degenerate and are subsequently re-absorbed. Relationships: is a type of developmental process involved in reproduction [GO:0003006]; is part of female gonad development [GO:0008585]; has part GO:0097191